{
  "gene_name": "Endophilin-B2",
  "gene_symbol": "SH3GLB2",
  "term_id": "GO:0006897",
  "gene": "UniProtKB:Q9NR46",
  "term_label": "endocytosis"
}